methyl transfer-driven active transmembrane transporter activity [GO:0015452] (molecular function) Also known as: Methyltransfer-driven transporters Relationships: is a type of GO:0015399; has part GO:0008168 Definition: Primary active transport of a solute across a membrane driven by a methyl transfer reaction. Primary active transport is catalysis of the transport of a solute across a membrane, up the solute's concentration gradient, by binding the solute and undergoing a series of conformational changes. Transport works equally well in either direction and is driven by a primary energy source. Sources: GOC:mtg_transport, ISBN:0815340729, TC:3.C.-.-.-